{
  "term_label": "dendrite membrane",
  "gene_symbol": "DAGLA",
  "gene": "UniProtKB:Q9Y4D2",
  "term_id": "GO:0032590",
  "gene_name": "Diacylglycerol lipase-alpha"
}